{
  "gene": "UniProtKB:Q96J02",
  "gene_symbol": "ITCH",
  "gene_name": "E3 ubiquitin-protein ligase Itchy homolog",
  "term_id": "GO:0043161",
  "term_label": "proteasome-mediated ubiquitin-dependent protein catabolic process"
}